{
  "term_label": "chloride:bicarbonate antiporter activity",
  "gene_name": "Anion exchange transporter",
  "gene_symbol": "SLC26A7",
  "term_id": "GO:0140900",
  "gene": "UniProtKB:Q8TE54"
}